chondrocyte activation [GO:0044566] (biological process) Relationships: is a type of cell activation [GO:0001775] Definition: A change in the morphology or behavior of a chondrocyte resulting from exposure to an activating factor such as a cellular or soluble ligand. A chondrocyte is a polymorphic cell that forms cartilage. Sources: CL:0000138, GOC:jl